{
  "term_id": "GO:0019970",
  "term_label": "interleukin-11 binding",
  "gene_symbol": "IL6R",
  "gene": "UniProtKB:P08887",
  "gene_name": "Interleukin-6 receptor subunit alpha"
}